{
  "gene_symbol": "OR9A1P",
  "term_label": "Unknown molecular function",
  "gene_name": "Olfactory receptor 9A1",
  "term_id": "UNKNOWN:0001",
  "gene": "UniProtKB:Q8NGU1"
}